{
  "gene": "UniProtKB:P59991",
  "term_label": "Unknown molecular function",
  "gene_symbol": "KRTAP12-2",
  "gene_name": "Keratin-associated protein 12-2",
  "term_id": "UNKNOWN:0001"
}